{
  "gene_name": "Frataxin, mitochondrial",
  "term_id": "GO:0008198",
  "gene_symbol": "FXN",
  "gene": "UniProtKB:Q16595",
  "term_label": "ferrous iron binding"
}